{
  "gene_symbol": "DHH",
  "gene": "UniProtKB:O43323",
  "gene_name": "Desert hedgehog protein",
  "term_label": "calcium ion binding",
  "term_id": "GO:0005509"
}